basal proximal dendrite [GO:0150017] (cellular component) Definition: Any dendrite in a dendritic tree that emerges near the basal pole of a neuron (e.g. in bipolar neurons, basal dendrites are either on the same side of the soma as the axon, or project toward the axon), and which is the closest to the cell body of the neuron (the soma). References: PMID:16899232, PMID:17046728, PMID:1720142, PMID:22683681, PMID:9214543 Sources: GOC:aruk, GOC:bc Relationships: is a type of basal dendrite [GO:0097441]; is a type of proximal dendrite [GO:1990635]